{
  "term_id": "GO:0004526",
  "gene": "UniProtKB:O15091",
  "gene_symbol": "PRORP",
  "gene_name": "Mitochondrial ribonuclease P catalytic subunit",
  "term_label": "ribonuclease P activity"
}